{
  "gene_symbol": "ZFPM2",
  "term_id": "GO:0030154",
  "term_label": "cell differentiation",
  "gene_name": "Zinc finger protein ZFPM2",
  "gene": "UniProtKB:Q8WW38"
}